{
  "gene_name": "Embryonic testis differentiation protein homolog B",
  "gene": "UniProtKB:P0DPP9",
  "gene_symbol": "ETDB",
  "term_label": "Unknown cellular component",
  "term_id": "UNKNOWN:0003"
}